{
  "gene_symbol": "RNF39",
  "term_id": "GO:0005737",
  "term_label": "cytoplasm",
  "gene_name": "RING finger protein 39",
  "gene": "UniProtKB:Q9H2S5"
}